{
  "term_label": "regulation of transcription by RNA polymerase II",
  "gene_symbol": "EBF1",
  "term_id": "GO:0006357",
  "gene": "UniProtKB:Q9UH73",
  "gene_name": "Transcription factor COE1"
}